{
  "term_label": "water channel activity",
  "gene_symbol": "AQP1",
  "gene_name": "Aquaporin-1",
  "gene": "UniProtKB:P29972",
  "term_id": "GO:0015250"
}